regulation of protein serine/threonine kinase activity [GO:0071900] (biological process) Relationships: is a type of GO:0045859; regulates protein serine/threonine kinase activity [GO:0004674] Definition: Any process that modulates the rate, frequency, or extent of protein serine/threonine kinase activity. Sources: GOC:mah Subtypes: GO:0000079, regulation of MAP kinase activity [GO:0043405], negative regulation of protein serine/threonine kinase activity [GO:0071901], positive regulation of protein serine/threonine kinase activity [GO:0071902], regulation of protein kinase C activity [GO:1900019], GO:2000298, regulation of cAMP-dependent protein kinase activity [GO:2000479]